glucose 6-phosphate:phosphate antiporter activity [GO:0061513] (molecular function) Relationships: is a type of glucose-6-phosphate transmembrane transporter activity [GO:0015152]; is_a hexose-phosphate:phosphate antiporter activity [GO:0015526] Also known as: glucose 6-phosphate:inorganic phosphate antiporter activity References: PMID:18337460 Sources: GOC:dph Definition: Enables the transfer of a solute or solutes from one side of a membrane to the other according to the reaction: glucose 6-phosphate(out) + phosphate(in) = glucose 6-phosphate(in) + phosphate(out).